{
  "term_label": "resolution of meiotic recombination intermediates",
  "term_id": "GO:0000712",
  "gene_name": "DNA repair endonuclease XPF",
  "gene": "UniProtKB:Q92889",
  "gene_symbol": "ERCC4"
}